{
  "gene_name": "Phytanoyl-CoA dioxygenase, peroxisomal",
  "term_id": "GO:0001561",
  "term_label": "fatty acid alpha-oxidation",
  "gene": "UniProtKB:O14832",
  "gene_symbol": "PHYH"
}